{
  "term_id": "GO:0036094",
  "gene_symbol": "AFP",
  "term_label": "small molecule binding",
  "gene_name": "Alpha-fetoprotein",
  "gene": "UniProtKB:P02771"
}